{
  "gene_name": "Tyrosine-protein phosphatase non-receptor type 1",
  "term_label": "cytoplasm",
  "gene": "UniProtKB:P18031",
  "term_id": "GO:0005737",
  "gene_symbol": "PTPN1"
}